{
  "gene_name": "Histone H3.1",
  "gene": "UniProtKB:P68431",
  "term_label": "nucleosomal DNA binding",
  "term_id": "GO:0031492",
  "gene_symbol": "H3C12"
}